{
  "gene": "UniProtKB:Q8N442",
  "term_id": "GO:0097177",
  "gene_name": "Translation factor GUF1, mitochondrial",
  "gene_symbol": "GUF1",
  "term_label": "mitochondrial ribosome binding"
}